ectopic germ cell programmed cell death [GO:0035234] (biological process) Also known as: programmed cell death of ectopic germ cells, programmed cell death, ectopic germ cells Relationships: is a type of developmental process involved in reproduction [GO:0003006]; is a type of GO:0010623 References: PMID:12814944 Definition: Programmed cell death of an errant germ line cell that is outside the normal migratory path or ectopic to the gonad. This is an important mechanism of regulating germ cell survival within the embryo.